{
  "term_id": "GO:0006886",
  "term_label": "intracellular protein transport",
  "gene": "UniProtKB:A4D1S5",
  "gene_name": "Ras-related protein Rab-19",
  "gene_symbol": "RAB19"
}